{
  "term_id": "GO:0034713",
  "gene_name": "TGF-beta receptor type-2",
  "gene_symbol": "TGFBR2",
  "term_label": "type I transforming growth factor beta receptor binding",
  "gene": "UniProtKB:P37173"
}